{
  "term_id": "GO:0007080",
  "gene_symbol": "H3-7",
  "gene": "UniProtKB:Q5TEC6",
  "gene_name": "Histone H3-7",
  "term_label": "mitotic metaphase chromosome alignment"
}